{
  "term_label": "extracellular space",
  "gene_symbol": "WFDC5",
  "term_id": "GO:0005615",
  "gene_name": "WAP four-disulfide core domain protein 5",
  "gene": "UniProtKB:Q8TCV5"
}